{
  "gene_symbol": "CLEC2A",
  "term_id": "GO:0005886",
  "gene": "UniProtKB:Q6UVW9",
  "gene_name": "C-type lectin domain family 2 member A",
  "term_label": "plasma membrane"
}